{
  "term_label": "Unknown cellular component",
  "term_id": "UNKNOWN:0003",
  "gene_name": "Retrotransposon Gag-like protein 8B",
  "gene": "UniProtKB:Q17RB0",
  "gene_symbol": "RTL8B"
}